{
  "term_label": "plasma membrane",
  "gene": "UniProtKB:Q9NV29",
  "term_id": "GO:0005886",
  "gene_symbol": "TMEM100",
  "gene_name": "Transmembrane protein 100"
}